tartronate O-hydroxycinnamoyltransferase activity [GO:0047161] (molecular function) Definition: Catalysis of the reaction: hydroxymalonate + sinapoyl-CoA = CoA + sinapoyltartronate. Sources: EC:2.3.1.106, RHEA:10952 Also known as: hydroxycinnamoyl-coenzyme-A:tartronate hydroxycinnamoyltransferase activity, sinapoyl-CoA:2-hydroxymalonate O-(hydroxycinnamoyl)transferase activity, tartronate sinapoyltransferase activity Relationships: is_a O-hydroxycinnamoyltransferase activity [GO:0050737]